cardiac left ventricle formation [GO:0003218] (biological process) Sources: GOC:mtg_heart Relationships: is a type of cardiac ventricle formation [GO:0003211]; is part of cardiac left ventricle morphogenesis [GO:0003214] Definition: The developmental process pertaining to the initial formation of a left cardiac ventricle from unspecified parts.